positive regulation of T-helper 17 cell extravasation [GO:2000457] (biological process) Definition: Any process that activates or increases the frequency, rate or extent of T-helper 17 cell extravasation. Sources: GOC:obol Relationships: is a type of positive regulation of CD8-positive, alpha-beta T cell extravasation [GO:2000451]; is a type of regulation of T-helper 17 cell extravasation [GO:2000455]; positively regulates GO:0035699